{
  "gene_name": "Glycine-rich extracellular protein 1",
  "term_label": "Unknown molecular function",
  "gene_symbol": "GREP1",
  "gene": "UniProtKB:A0A0J9YXV3",
  "term_id": "UNKNOWN:0001"
}